{
  "term_label": "plasma membrane",
  "gene_symbol": "SLC39A4",
  "gene": "UniProtKB:Q6P5W5",
  "gene_name": "Zinc transporter ZIP4",
  "term_id": "GO:0005886"
}